{
  "term_label": "Ku70:Ku80 complex",
  "gene": "UniProtKB:P13010",
  "gene_symbol": "XRCC5",
  "gene_name": "X-ray repair cross-complementing protein 5",
  "term_id": "GO:0043564"
}